{
  "term_label": "nucleus",
  "gene_name": "Cullin-3",
  "term_id": "GO:0005634",
  "gene_symbol": "CUL3",
  "gene": "UniProtKB:Q13618"
}